{
  "term_id": "GO:0005886",
  "gene": "UniProtKB:Q8IZJ4",
  "gene_symbol": "RGL4",
  "gene_name": "Ral-GDS-related protein",
  "term_label": "plasma membrane"
}